{
  "term_id": "GO:1990275",
  "gene_name": "Nuclear valosin-containing protein-like",
  "term_label": "preribosome binding",
  "gene_symbol": "NVL",
  "gene": "UniProtKB:O15381"
}